{
  "term_id": "GO:0036128",
  "term_label": "CatSper complex",
  "gene": "UniProtKB:Q8NEC5",
  "gene_name": "Cation channel sperm-associated protein 1",
  "gene_symbol": "CATSPER1"
}